{
  "gene": "UniProtKB:Q96HC4",
  "gene_name": "PDZ and LIM domain protein 5",
  "term_id": "GO:0003779",
  "term_label": "actin binding",
  "gene_symbol": "PDLIM5"
}